{
  "gene": "UniProtKB:P01570",
  "term_id": "GO:0002286",
  "gene_symbol": "IFNA14",
  "term_label": "T cell activation involved in immune response",
  "gene_name": "Interferon alpha-14"
}